{
  "gene_name": "Nuclear pore complex-interacting protein family member A8",
  "gene": "UniProtKB:P0DM63",
  "gene_symbol": "NPIPA8",
  "term_id": "UNKNOWN:0001",
  "term_label": "Unknown molecular function"
}